{
  "gene_symbol": "PLCB4",
  "term_label": "phosphatidylinositol-mediated signaling",
  "gene": "UniProtKB:Q15147",
  "term_id": "GO:0048015",
  "gene_name": "1-phosphatidylinositol 4,5-bisphosphate phosphodiesterase beta-4"
}